polymeric immunoglobulin receptor activity [GO:0001792] (molecular function) Sources: GOC:add, GOC:signaling, ISBN:0781735149 Relationships: is a type of immunoglobulin receptor activity [GO:0019763]; has part GO:0001790 Definition: Combining with a J-chain-containing polymeric immunoglobulin of the IgA or IgM isotypes via the Fc region, and transmitting the signal from one side of the membrane to the other to initiate a change in cell activity.